{
  "gene_name": "XK-related protein 9",
  "term_id": "GO:0016020",
  "gene": "UniProtKB:Q5GH70",
  "term_label": "membrane",
  "gene_symbol": "XKR9"
}